{
  "gene_name": "Hexokinase-3",
  "term_id": "GO:0005829",
  "gene": "UniProtKB:P52790",
  "term_label": "cytosol",
  "gene_symbol": "HK3"
}